{
  "term_label": "Unknown biological process",
  "term_id": "UNKNOWN:0002",
  "gene_name": "Putative uncharacterized protein encoded by LINC00479",
  "gene": "UniProtKB:Q96M42",
  "gene_symbol": "LINC00479"
}